{
  "term_id": "GO:0003723",
  "gene": "UniProtKB:Q8IY67",
  "gene_symbol": "RAVER1",
  "term_label": "RNA binding",
  "gene_name": "Ribonucleoprotein PTB-binding 1"
}